{
  "gene_symbol": "TBX19",
  "term_id": "GO:0005634",
  "gene": "UniProtKB:O60806",
  "term_label": "nucleus",
  "gene_name": "T-box transcription factor TBX19"
}